{
  "term_id": "GO:0070989",
  "term_label": "oxidative demethylation",
  "gene_name": "Cytochrome P450 3A43",
  "gene_symbol": "CYP3A43",
  "gene": "UniProtKB:Q9HB55"
}